{
  "term_id": "GO:0030893",
  "gene": "UniProtKB:Q8NDV3",
  "term_label": "meiotic cohesin complex",
  "gene_name": "Structural maintenance of chromosomes protein 1B",
  "gene_symbol": "SMC1B"
}